(3S,4R)-3,4-dihydroxycyclohexa-1,5-diene-1,4-dicarboxylate dehydrogenase activity [GO:0047120] (molecular function) Definition: Catalysis of the reaction: (3S,4R)-3,4-dihydroxycyclohexa-1,5-diene-1,4-dicarboxylate + NAD+ = 3,4-dihydroxybenzoate + CO2 + NADH. Sources: EC:1.3.1.53, RHEA:10744 Also known as: terephthalate 1,2-cis-dihydrodiol dehydrogenase activity, (1R,2S)-dihydroxy-3,5-cyclohexadiene-1,4-dicarboxylate dehydrogenase activity, (3S,4R)-3,4-dihydroxycyclohexa-1,5-diene-1,4-dicarboxylate:NAD+ oxidoreductase activity, cis-4,5-dihydroxycyclohexa-1(6),2-diene-1,4-dicarboxylate:NAD+ oxidoreductase (decarboxylating), dihydroxy-3,5-cyclohexadiene-1,4-dicarboxylate dehydrogenase activity Relationships: is a type of GO:0016628